regulation of maltotetraose transport [GO:1900321] (biological process) Subtypes: GO:1900322, GO:1900323 Relationships: is a type of regulation of transport [GO:0051049]; regulates maltotetraose transport [GO:2001099] Definition: Any process that modulates the frequency, rate or extent of maltotetraose transport. Sources: GOC:TermGenie, GOC:mengo_curators